ligase activity [GO:0016874] (molecular function) Regulation: positively regulated by GO:0051351; regulated by ligase regulator activity [GO:0055103]; negatively regulated by GO:0055104 Relationships: is a type of GO:0003824 Also known as: synthetase activity Definition: Catalysis of the joining of two molecules, or two groups within a single molecule, using the energy from the hydrolysis of ATP, a similar triphosphate, or a pH gradient. Sources: EC:6.-.-.- Subtypes: ligase activity, forming carbon-oxygen bonds [GO:0016875], GO:0016877, ligase activity, forming carbon-nitrogen bonds [GO:0016879], ligase activity, forming carbon-carbon bonds [GO:0016885], ligase activity, forming phosphoric ester bonds [GO:0016886], sodium-transporting ATP synthase activity, rotational mechanism [GO:0046932], proton-transporting ATP synthase activity, rotational mechanism [GO:0046933], ligase activity, forming nitrogen-metal bonds [GO:0051002]